sex chromatin [GO:0001739] (cellular component) Sources: GOC:dos, ISBN:0198506732 Relationships: is a type of GO:0000792; is part of GO:0000803 Subtypes: condensed chromatin of inactivated sex chromosome [GO:0098578] Definition: Chromatin that is part of a sex chromosome.